tRNA (cytidine-5-)-methyltransferase activity [GO:0016428] (molecular function) Relationships: is_a tRNA (cytidine) methyltransferase activity [GO:0016427] Definition: Catalysis of the reaction: a cytidine in tRNA + S-adenosyl-L-methionine = a 5-methylcytidine in tRNA + S-adenosyl-L-homocysteine + H+. This modification can occur on seversal residues, including cytidine(34), cytidine(40), cytidine(48), and cytidine(49). Also known as: tRNA (cytosine-5-)-methyltransferase activity, S-adenosyl-L-methionine:tRNA (cytosine-5-)-methyltransferase activity, transfer RNA cytosine 5-methyltransferase activity, transfer ribonucleate cytosine 5-methyltransferase activity Sources: RHEA:61468